{
  "gene": "UniProtKB:P83859",
  "term_id": "GO:0031854",
  "term_label": "orexigenic neuropeptide QRFP receptor binding",
  "gene_name": "Orexigenic neuropeptide QRFP",
  "gene_symbol": "QRFP"
}